{
  "term_id": "UNKNOWN:0002",
  "term_label": "Unknown biological process",
  "gene_symbol": "FOLH1B",
  "gene": "UniProtKB:Q9HBA9",
  "gene_name": "Putative N-acetylated-alpha-linked acidic dipeptidase"
}